peptidyl-lysine hydroxylation [GO:0017185] (biological process) Relationships: is_a protein hydroxylation [GO:0018126]; is a type of peptidyl-lysine modification [GO:0018205] Sources: GOC:ai Definition: The hydroxylation of peptidyl-lysine to form peptidyl-hydroxylysine. Subtypes: GO:0018395